{
  "term_label": "T cell receptor signaling pathway",
  "gene": "UniProtKB:Q13410",
  "gene_symbol": "BTN1A1",
  "term_id": "GO:0050852",
  "gene_name": "Butyrophilin subfamily 1 member A1"
}